{
  "term_label": "sensory perception of chemical stimulus",
  "term_id": "GO:0007606",
  "gene_symbol": "GNAS",
  "gene": "UniProtKB:Q5JWF2",
  "gene_name": "Guanine nucleotide-binding protein G(s) subunit alpha isoforms XLas"
}